{
  "gene_symbol": "CLIC4",
  "term_label": "cytoplasm",
  "term_id": "GO:0005737",
  "gene": "UniProtKB:Q9Y696",
  "gene_name": "Chloride intracellular channel protein 4"
}